{
  "gene_symbol": "GBP6",
  "gene": "UniProtKB:Q6ZN66",
  "term_id": "GO:0071346",
  "gene_name": "Guanylate-binding protein 6",
  "term_label": "cellular response to type II interferon"
}